{
  "gene_symbol": "SLC7A13",
  "gene_name": "Solute carrier family 7 member 13",
  "term_id": "GO:0003333",
  "term_label": "amino acid transmembrane transport",
  "gene": "UniProtKB:Q8TCU3"
}